compound sieve plate [GO:0097219] (cellular component) Relationships: is a type of GO:0097218 Definition: A sieve plate that contains several specialized sieve areas in either a scalariform or reticulate arrangement. Sources: ISBN:0471738433, POC:curators Note: Often located on an end wall of a sieve tube member. Unspecialized sieve areas may occur on other parts of the cell.